kinetochore assembly [GO:0051382] (BP) Regulation: regulated by regulation of kinetochore assembly [GO:0090234]; negatively regulated by negative regulation of kinetochore assembly [GO:1905560]; positively regulated by positive regulation of kinetochore assembly [GO:1905561] Also known as: NMS complex assembly, centromere and kinetochore complex maturation, centromere/kinetochore complex maturation, chromosome-kinetochore attachment, kinetochore formation Definition: The aggregation, arrangement and bonding together of a set of components to form the kinetochore, a multisubunit complex that is located at the centromeric region of DNA and provides an attachment point for the spindle microtubules. Relationships: is a type of kinetochore organization [GO:0051383]; is a type of protein-containing complex assembly [GO:0065003]; is_a membraneless organelle assembly [GO:0140694] Sources: GOC:ai